{
  "gene": "UniProtKB:A6QL64",
  "gene_name": "Ankyrin repeat domain-containing protein 36A",
  "gene_symbol": "ANKRD36",
  "term_label": "Unknown biological process",
  "term_id": "UNKNOWN:0002"
}